{
  "term_id": "GO:0050829",
  "term_label": "defense response to Gram-negative bacterium",
  "gene": "UniProtKB:P18428",
  "gene_symbol": "LBP",
  "gene_name": "Lipopolysaccharide-binding protein"
}